viral budding via host ESCRT complex [GO:0039702] (biological process) Relationships: is a type of viral budding [GO:0046755] Sources: UniProtKB-KW:KW-1187, VZ:1536 Regulation: regulated by regulation of viral budding via host ESCRT complex [GO:1903772]; negatively regulated by negative regulation of viral budding via host ESCRT complex [GO:1903773]; positively regulated by positive regulation of viral budding via host ESCRT complex [GO:1903774] Definition: Viral budding which uses a host ESCRT protein complex, or complexes, to mediate the budding process. Also known as: host-assisted viral budding, viral budding through the ESCRT machinery